intracellularly gated calcium channel activity [GO:0015278] (molecular function) Sources: GOC:mah Also known as: calcium-release channel activity, intracellular ligand-gated calcium channel activity Relationships: is a type of intracellularly ligand-gated monoatomic ion channel activity [GO:0005217]; is a type of ligand-gated calcium channel activity [GO:0099604] Definition: Enables the transmembrane transfer of a calcium ion by a channel that opens when a specific intracellular ligand has been bound by the channel complex or one of its constituent parts. Subtypes: inositol 1,4,5-trisphosphate-gated calcium channel activity [GO:0005220], calcium-induced calcium release activity [GO:0048763], NAADP-sensitive calcium-release channel activity [GO:0072345], cADPR-sensitive calcium-release channel activity [GO:0072346], intracellularly ATP-gated calcium channel activity [GO:0140417]